{
  "gene": "UniProtKB:Q5TGP6",
  "term_label": "Unknown cellular component",
  "term_id": "UNKNOWN:0003",
  "gene_name": "Maestro heat-like repeat-containing protein family member 9",
  "gene_symbol": "MROH9"
}